His-Purkinje system development [GO:0003164] (biological process) Definition: The process whose specific outcome is the progression of the His-Purkinje system over time, from its formation to the mature structure. The His-Purkinje system receives signals from the AV node and is composed of the fibers that regulate cardiac muscle contraction in the ventricles. Sources: GOC:mtg_heart Relationships: is a type of ventricular cardiac muscle tissue development [GO:0003229]; is part of cardiac conduction system development [GO:0003161]